{
  "term_id": "GO:0000122",
  "gene": "UniProtKB:P41182",
  "gene_name": "B-cell lymphoma 6 protein",
  "gene_symbol": "BCL6",
  "term_label": "negative regulation of transcription by RNA polymerase II"
}